{
  "gene_name": "Heat shock 70 kDa protein 6",
  "gene_symbol": "HSPA6",
  "gene": "UniProtKB:P17066",
  "term_id": "GO:0016887",
  "term_label": "ATP hydrolysis activity"
}